{
  "term_id": "GO:0005737",
  "gene_name": "SAM domain-containing protein SAMSN-1",
  "gene": "UniProtKB:Q9NSI8",
  "gene_symbol": "SAMSN1",
  "term_label": "cytoplasm"
}